{
  "term_label": "myelination",
  "term_id": "GO:0042552",
  "gene_symbol": "BCAS1",
  "gene_name": "Breast carcinoma-amplified sequence 1",
  "gene": "UniProtKB:O75363"
}